{
  "gene_symbol": "PRKACA",
  "gene_name": "cAMP-dependent protein kinase catalytic subunit alpha",
  "term_id": "GO:0005829",
  "gene": "UniProtKB:P17612",
  "term_label": "cytosol"
}